{
  "gene": "UniProtKB:P0C7P4",
  "term_label": "mitochondrial electron transport, ubiquinol to cytochrome c",
  "term_id": "GO:0006122",
  "gene_name": "Putative cytochrome b-c1 complex subunit Rieske-like protein 1",
  "gene_symbol": "UQCRFS1P1"
}